positive regulation of ergosterol biosynthetic process [GO:0070452] (biological process) Definition: Any process that activates or increases the frequency, rate or extent of the chemical reactions and pathways resulting in the formation of ergosterol. Sources: GOC:mah Relationships: is a type of GO:0032443; is a type of GO:0106120; is a type of positive regulation of alcohol biosynthetic process [GO:1902932]; RO_0002213 GO:0006696 Also known as: positive regulation of ergosterol anabolism, positive regulation of ergosterol biosynthesis, positive regulation of ergosterol formation, positive regulation of ergosterol synthesis, up regulation of ergosterol biosynthetic process, up-regulation of ergosterol biosynthetic process, upregulation of ergosterol biosynthetic process, activation of ergosterol biosynthetic process, stimulation of ergosterol biosynthetic process